{
  "gene_name": "Nucleotide sugar transporter SLC35D1",
  "term_label": "UDP-N-acetylglucosamine transmembrane transporter activity",
  "gene": "UniProtKB:Q9NTN3",
  "term_id": "GO:0005462",
  "gene_symbol": "SLC35D1"
}